{
  "gene_name": "ATP-dependent Clp protease ATP-binding subunit clpX-like, mitochondrial",
  "term_id": "GO:0005524",
  "gene": "UniProtKB:O76031",
  "gene_symbol": "CLPX",
  "term_label": "ATP binding"
}